{
  "term_id": "UNKNOWN:0003",
  "gene_symbol": "CTDNEP1",
  "gene": "UniProtKB:O95476",
  "gene_name": "CTD nuclear envelope phosphatase 1",
  "term_label": "Unknown cellular component"
}